metanephric comma-shaped body morphogenesis [GO:0072278] (biological process) Relationships: is a type of comma-shaped body morphogenesis [GO:0072049]; BFO_0000050 metanephric nephron morphogenesis [GO:0072273] Sources: GOC:mtg_kidney_jan10 Regulation: regulated by regulation of metanephric comma-shaped body morphogenesis [GO:2000006]; RO_0002212 by negative regulation of metanephric comma-shaped body morphogenesis [GO:2000007] Definition: The process in which the metanephric comma-shaped body is generated and organized. The metanephric comma-shaped body is the precursor structure to the metanephric S-shaped body that contributes to the morphogenesis of a nephron in the metanephros.